3-hydroxy-3-isohexenylglutaryl-CoA lyase activity [GO:0047445] (molecular function) Definition: Catalysis of the reaction: 3-hydroxy-3-(4-methylpent-3-en-1-yl)glutaryl-CoA + 4 H+ = 7-methyl-3-oxooct-6-enoyl-CoA + acetate. Sources: EC:4.1.3.26, RHEA:23084 Also known as: 3-hydroxy-3-(4-methylpent-3-en-1-yl)glutaryl-CoA acetate-lyase (7-methyl-3-oxooct-6-enoyl-CoA-forming), 3-hydroxy-3-(4-methylpent-3-en-1-yl)glutaryl-CoA acetate-lyase activity, 3-hydroxy-3-isohexenylglutaryl coenzyme A lyase activity, 3-hydroxy-3-isohexenylglutaryl-CoA isopentenylacetoacetyl-CoA-lyase activity, beta-hydroxy-beta-isohexenylglutaryl CoA-lyase activity, hydroxyisohexenylglutaryl-CoA:acetatelyase activity Relationships: is a type of GO:0016833